{
  "gene_symbol": "CFAP91",
  "term_label": "Unknown cellular component",
  "term_id": "UNKNOWN:0003",
  "gene": "UniProtKB:Q7Z4T9",
  "gene_name": "Cilia- and flagella-associated protein 91"
}